snoRNA transcription by RNA polymerase II [GO:0001015] (biological process) Definition: The synthesis of small nucleolar RNA (snoRNA) from a DNA template by RNA polymerase II, originating at an RNA polymerase II promoter. Relationships: is_a GO:0006366; is a type of sno(s)RNA transcription [GO:0009302] Sources: GOC:txnOH Also known as: snoRNA transcription from an RNA polymerase II promoter